UDP-N-acetylglucosamine-dolichyl-phosphate N-acetylglucosaminephosphotransferase activity [GO:0003975] (molecular function) Definition: Catalysis of the reaction: UDP-N-acetyl-D-glucosamine + dolichyl phosphate = UMP + N-acetyl-D-glucosaminyl-diphosphodolichol. Also known as: UDP-N-acetylglucosamine-dolichyl-phosphate N-acetylglucosamine-1-phosphate transferase activity, GlcNAc-1-P transferase activity, N-acetylglucosamine-1-phosphate transferase activity, UDP-D-N-acetylglucosamine N-acetylglucosamine 1-phosphate transferase activity, UDP-GlcNAc:dolichyl-phosphate GlcNAc-1-phosphate transferase activity, UDP-N-acetyl-D-glucosamine:dolichol phosphate N-acetyl-D-glucosamine-1-phosphate transferase activity, UDP-N-acetyl-D-glucosamine:dolichyl-phosphate N-acetyl-D-glucosaminephosphotransferase activity, UDP-acetylglucosamine-dolichol phosphate acetylglucosamine phosphotransferase activity, UDP-acetylglucosamine-dolichol phosphate acetylglucosamine-1-phosphotransferase activity, chitobiosylpyrophosphoryldolichol synthase activity, dolichol phosphate N-acetylglucosamine-1-phosphotransferase activity, uridine diphosphoacetylglucosamine-dolichyl phosphate acetylglucosamine-1-phosphotransferase activity Sources: EC:2.7.8.15 Relationships: is a type of phosphotransferase activity, for other substituted phosphate groups [GO:0016780]